{
  "term_id": "GO:0006357",
  "gene_name": "Sp110 nuclear body protein",
  "gene_symbol": "SP110",
  "term_label": "regulation of transcription by RNA polymerase II",
  "gene": "UniProtKB:Q9HB58"
}